{
  "gene": "UniProtKB:Q8TDW7",
  "term_label": "plasma membrane",
  "gene_name": "Protocadherin Fat 3",
  "term_id": "GO:0005886",
  "gene_symbol": "FAT3"
}